satellite fibril [GO:0071808] (cellular component) References: PMID:20108326 Sources: GOC:mah, GOC:sl Definition: An axoneme part that is found in the flagella of mammalian sperm and is located in the middle piece between the outer dense fibers (on the concave side of outer dense fibers as seen in cross-section). Relationships: is a type of cellular anatomical structure [GO:0110165]; is part of axoneme [GO:0005930]